{
  "term_id": "GO:0006357",
  "gene_symbol": "ZNF395",
  "term_label": "regulation of transcription by RNA polymerase II",
  "gene_name": "Zinc finger protein 395",
  "gene": "UniProtKB:Q9H8N7"
}